{
  "gene_name": "Golgin subfamily A member 6-like protein 2",
  "gene": "UniProtKB:Q8N9W4",
  "gene_symbol": "GOLGA6L2",
  "term_label": "Unknown biological process",
  "term_id": "UNKNOWN:0002"
}